{
  "term_id": "GO:0030291",
  "gene_symbol": "INKA1",
  "gene": "UniProtKB:Q96EL1",
  "gene_name": "PAK4-inhibitor INKA1",
  "term_label": "protein serine/threonine kinase inhibitor activity"
}